analia morphogenesis [GO:0048809] (biological process) Definition: The process in which the anatomical structures of analia are generated and organized. The analia is the posterior-most vertral appendage that develops from the genital disc. An example of this process is analia morphogenesis in Drosophila melanogaster. Sources: GOC:ai, GOC:mtg_sensu Subtypes: female analia morphogenesis [GO:0048810], GO:0048811 Relationships: is a type of post-embryonic animal morphogenesis [GO:0009886]; is part of GO:0007483; is part of GO:0007487